cyanohydrin beta-glucosyltransferase activity [GO:0047792] (molecular function) Sources: EC:2.4.1.85 Relationships: is a type of UDP-glucosyltransferase activity [GO:0035251] Also known as: cyanohydrin b-glucosyltransferase activity, UGT85B1 activity, UDP-D-glucose:(S)-4-hydroxymandelonitrile beta-D-glucosyltransferase activity, UDP-glucose-p-hydroxymandelonitrile glucosyltransferase activity, UDP-glucose:(S)-4-hydroxymandelonitrile beta-D-glucosyltransferase activity, UDP-glucose:p-hydroxymandelonitrile-O-glucosyltransferase activity, uridine diphosphoglucose-cyanohydrin glucosyltransferase activity, uridine diphosphoglucose-p-hydroxymandelonitrile glucosyltransferase activity, uridine diphosphoglucose:aldehyde cyanohydrin beta-glucosyltransferase activity Definition: Catalysis of the reaction: UDP-glucose + (S)-4-hydroxymandelonitrile = UDP + (S)-4-hydroxy-mandelonitrile beta-D-glucoside.